{
  "gene_symbol": "COG5",
  "gene_name": "Conserved oligomeric Golgi complex subunit 5",
  "gene": "UniProtKB:Q9UP83",
  "term_id": "UNKNOWN:0001",
  "term_label": "Unknown molecular function"
}